phospholipase C/protein kinase C signal transduction [GO:0141212] (biological process) Also known as: PLC/PKC signaling, PLC/PKC/PKD signaling Definition: An intracellular signaling cassette that starts with activation of phospholipase C (PLC) activity and ends with the activation of protein kinase C (PKC). PLC produces inositol 1,4,5-trisphosphate (IP3) and diacylglycerol (DAG). IP3 regulates the opening of calcium channels in intracellular calcium store, leading to the release of calcium into the cytosol. Calcium and DAG activate protein kinase C (PKC), which in turn activates downstream effectors. This cassette is often part of the phospholipase C-activating G protein-coupled receptor signaling pathway. Regulation: positively regulated by positive regulation of phospholipase C/protein kinase C signal transduction [GO:0141214]; negatively regulated by negative regulation of phospholipase C/protein kinase C signal transduction [GO:0160195] Relationships: is a type of intracellular signaling cassette [GO:0141124] References: PMID:26605346